{
  "term_label": "nuclear mRNA surveillance",
  "term_id": "GO:0071028",
  "gene_name": "Exosome complex component RRP41",
  "gene_symbol": "EXOSC4",
  "gene": "UniProtKB:Q9NPD3"
}